{
  "gene_symbol": "MRAP2",
  "gene_name": "Melanocortin-2 receptor accessory protein 2",
  "term_label": "endoplasmic reticulum",
  "term_id": "GO:0005783",
  "gene": "UniProtKB:Q96G30"
}